regulation of protein processing involved in protein targeting to mitochondrion [GO:1903216] (biological process) Relationships: is a type of GO:0070613; regulates protein processing involved in protein targeting to mitochondrion [GO:0006627] Also known as: regulation of mitochondrial processing, regulation of mitochondrial protein processing during import References: PMID:21370995 Sources: GOC:PARL, GOC:TermGenie, GOC:bf, GO_REF:0000058 Definition: Any process that modulates the frequency, rate or extent of protein processing involved in protein targeting to mitochondrion. Subtypes: negative regulation of protein processing involved in protein targeting to mitochondrion [GO:1903217]